{
  "gene_name": "Thioredoxin domain-containing protein 3",
  "term_label": "sperm principal piece",
  "term_id": "GO:0097228",
  "gene_symbol": "NME8",
  "gene": "UniProtKB:Q8N427"
}